{
  "gene": "UniProtKB:P09471",
  "term_label": "cytoplasm",
  "gene_symbol": "GNAO1",
  "gene_name": "Guanine nucleotide-binding protein G(o) subunit alpha",
  "term_id": "GO:0005737"
}